{
  "gene": "UniProtKB:P09496",
  "term_id": "GO:0030672",
  "gene_name": "Clathrin light chain A",
  "term_label": "synaptic vesicle membrane",
  "gene_symbol": "CLTA"
}